{
  "gene_name": "Transient receptor potential cation channel subfamily M member 2",
  "term_label": "ligand-gated calcium channel activity",
  "gene_symbol": "TRPM2",
  "gene": "UniProtKB:O94759",
  "term_id": "GO:0099604"
}